{
  "gene_name": "Cyclin N-terminal domain-containing protein 1",
  "gene": "UniProtKB:Q8N815",
  "term_label": "site of double-strand break",
  "gene_symbol": "CNTD1",
  "term_id": "GO:0035861"
}